{
  "gene_name": "Heterogeneous nuclear ribonucleoprotein L",
  "term_id": "GO:0043484",
  "term_label": "regulation of RNA splicing",
  "gene_symbol": "HNRNPL",
  "gene": "UniProtKB:P14866"
}